{
  "term_label": "hormone activity",
  "term_id": "GO:0005179",
  "gene_name": "Chorionic somatomammotropin hormone 1",
  "gene": "UniProtKB:P0DML2",
  "gene_symbol": "CSH1"
}